developmental process involved in reproduction [GO:0003006] (biological process) Also known as: puberty, reproductive developmental process Sources: GOC:dph, GOC:isa_complete Definition: A developmental process in which a progressive change in the state of some part of an organism, germline or somatic, specifically contributes to its ability to form offspring. Relationships: is a type of reproductive process [GO:0022414]; is a type of GO:0032502 Subtypes: antral ovarian follicle growth [GO:0001547], GO:0001549, GO:0001552, GO:0001555, oocyte maturation [GO:0001556], acrosome assembly [GO:0001675], Mullerian duct regression [GO:0001880], GO:0001893, GO:0007277, pole cell fate determination [GO:0007278], pole cell formation [GO:0007279], germ cell development [GO:0007281], spermatogenesis [GO:0007283], primary spermatocyte growth [GO:0007285], Nebenkern assembly [GO:0007287], sperm axoneme assembly [GO:0007288], sperm individualization [GO:0007291], germarium-derived egg chamber formation [GO:0007293], GO:0007294, GO:0007295, egg chorion assembly [GO:0007306], oocyte construction [GO:0007308], oocyte axis specification [GO:0007309], gonadal mesoderm development [GO:0007506], GO:0007530, donor selection [GO:0007535], sex determination, establishment of X:A ratio [GO:0007540], sex determination, primary response to X:A ratio [GO:0007541], sex differentiation [GO:0007548], dorsal/ventral axis specification, ovarian follicular epithelium [GO:0008069], GO:0009560, embryo development ending in seed dormancy [GO:0009793], GO:0009860, longitudinal axis specification [GO:0009942], GO:0009960, oocyte differentiation [GO:0009994], root meristem specification [GO:0010071], GO:0010072, GO:0010093, GO:0010162, GO:0010198, GO:0010214, GO:0010227, vegetative to reproductive phase transition of meristem [GO:0010228], anther wall tapetum cell fate specification [GO:0010234], GO:0010254, GO:0010431, inflorescence meristem growth [GO:0010450], floral meristem growth [GO:0010451], microsporocyte differentiation [GO:0010480], GO:0010582, GO:0010622, apical cell fate commitment [GO:0010654], chorion-containing eggshell pattern formation [GO:0030381], asexual sporulation [GO:0030436], ascospore wall assembly [GO:0030476], GO:0030703, vitelline membrane formation [GO:0030704], GO:0030707, GO:0030713, GO:0030714, ascospore-type prospore assembly [GO:0031321], ascospore-type prospore membrane formation [GO:0032120], Leydig cell differentiation [GO:0033327], sexual sporulation [GO:0034293], sexual spore wall assembly [GO:0034294], centrosomal and pronuclear rotation [GO:0035047], genitalia morphogenesis [GO:0035112], GO:0035234, gonad morphogenesis [GO:0035262], genital disc sexually dimorphic development [GO:0035263], GO:0035846, asexual spore wall assembly [GO:0042243], menstrual cycle [GO:0044850], development of secondary sexual characteristics [GO:0045136], GO:0045137, nurse cell apoptotic process [GO:0045476], decidualization [GO:0046697], dorsal appendage formation [GO:0046843], chorion micropyle formation [GO:0046844], GO:0048071, germ-line cyst encapsulation [GO:0048138], pollen sperm cell differentiation [GO:0048235], GO:0048240, inflorescence morphogenesis [GO:0048281], GO:0048317, GO:0048437, floral whorl development [GO:0048438], GO:0048439, floral organ morphogenesis [GO:0048444], floral organ formation [GO:0048449], floral whorl morphogenesis [GO:0048457], GO:0048458, GO:0048459, flower formation [GO:0048460], flower structural organization [GO:0048461], style development [GO:0048479], stigma development [GO:0048480], plant ovule development [GO:0048481], plant ovule morphogenesis [GO:0048482], embryonic meristem development [GO:0048508], spermatid differentiation [GO:0048515], fruit morphogenesis [GO:0048530], establishment of floral organ orientation [GO:0048559], oocyte fate commitment [GO:0048600], oocyte morphogenesis [GO:0048601], reproductive structure development [GO:0048608], GO:0048624, anther development [GO:0048653], anther wall tapetum morphogenesis [GO:0048655], anther wall tapetum formation [GO:0048656], GO:0048657, anther wall tapetum development [GO:0048658], acquisition of desiccation tolerance in seed [GO:0048700], specification of floral organ number [GO:0048833], pollen tube development [GO:0048868], Sertoli cell differentiation [GO:0060008], Sertoli cell development [GO:0060009], Sertoli cell fate commitment [GO:0060010], GO:0060512, prostate field specification [GO:0060515], dichotomous subdivision of prostate epithelial cord terminal unit [GO:0060524], prostate glandular acinus development [GO:0060525], GO:0060530, cell differentiation involved in embryonic placenta development [GO:0060706], prostate gland growth [GO:0060736], prostate gland epithelium morphogenesis [GO:0060740], prostate gland stromal morphogenesis [GO:0060741], epithelial cell differentiation involved in prostate gland development [GO:0060742], mammary gland branching involved in pregnancy [GO:0060745], tertiary branching involved in mammary gland duct morphogenesis [GO:0060748], uterus morphogenesis [GO:0061038], seminal vesicle epithelium development [GO:0061108], paramesonephric duct development [GO:0061205], conidiophore stalk development [GO:0070788], metula development [GO:0070789], phialide development [GO:0070790], Hulle cell development [GO:0070792], ascospore release from ascus [GO:0071998], integument development [GO:0080060], stamen filament development [GO:0080086], GO:0080126, fruit septum development [GO:0080127], GO:0080128, stomium development [GO:0080166], GO:0090376, seed trichome initiation [GO:0090377], seed trichome elongation [GO:0090378], seed trichome maturation [GO:0090380], GO:0120316, spermatid cytoplasm removal during spermiation of flagellated sperm [GO:0160087]